{
  "term_label": "FACT complex",
  "term_id": "GO:0035101",
  "gene_name": "FACT complex subunit SSRP1",
  "gene": "UniProtKB:Q08945",
  "gene_symbol": "SSRP1"
}